{
  "gene": "UniProtKB:Q6UWP7",
  "term_id": "GO:0036149",
  "gene_symbol": "LCLAT1",
  "gene_name": "Lysocardiolipin acyltransferase 1",
  "term_label": "phosphatidylinositol acyl-chain remodeling"
}